{
  "term_label": "DNA binding",
  "gene": "UniProtKB:P51531",
  "gene_symbol": "SMARCA2",
  "term_id": "GO:0003677",
  "gene_name": "Probable global transcription activator SNF2L2"
}